{
  "gene_symbol": "LIAT1",
  "gene": "UniProtKB:Q6ZQX7",
  "term_label": "Unknown biological process",
  "term_id": "UNKNOWN:0002",
  "gene_name": "Protein LIAT1"
}